{
  "term_label": "intracellular protein transport",
  "gene": "UniProtKB:P84077",
  "gene_symbol": "ARF1",
  "gene_name": "ADP-ribosylation factor 1",
  "term_id": "GO:0006886"
}